{
  "gene": "UniProtKB:Q8NGK5",
  "term_id": "GO:0005886",
  "term_label": "plasma membrane",
  "gene_symbol": "OR52M1",
  "gene_name": "Olfactory receptor 52M1"
}